nicotianamine catabolic process [GO:0030419] (biological process) Definition: The chemical reactions and pathways resulting in the breakdown of nicotianamine, 2(S),3'2(S),3''(S)-N-(N-(3-amino-3-carboxypropyl)-3-amino-3-carboxypropyl)-azetidine-2-carboxylic acid. Relationships: is a type of amino acid catabolic process [GO:0009063]; is a type of biogenic amine catabolic process [GO:0042402]; is a type of tricarboxylic acid catabolic process [GO:0072352] References: PMID:10069850 Sources: GOC:mah Also known as: nicotianamine breakdown, nicotianamine catabolism, nicotianamine degradation